{
  "term_label": "lipid metabolic process",
  "gene_symbol": "LIPJ",
  "gene_name": "Lipase member J",
  "term_id": "GO:0006629",
  "gene": "UniProtKB:Q5W064"
}